replication fork arrest involved in DNA replication termination [GO:0071807] (biological process) Relationships: is a type of replication fork arrest [GO:0043111]; is part of DNA replication termination [GO:0006274] References: PMID:17347517, PMID:20797631 Sources: GOC:mah Definition: A replication fork arrest process that contributes to the termination of DNA replication.